tRNA demethylase activity [GO:1990984] (molecular function) Relationships: is a type of oxidative RNA demethylase activity [GO:0035515]; is_a catalytic activity, acting on a tRNA [GO:0140101] Definition: Catalysis of the removal of a methyl group from one or more positions within a tRNA molecule. References: PMID:27745969